{
  "gene": "UniProtKB:Q96MW5",
  "gene_name": "Conserved oligomeric Golgi complex subunit 8",
  "term_label": "Golgi transport complex",
  "term_id": "GO:0017119",
  "gene_symbol": "COG8"
}